{
  "gene_name": "NEDD4-binding protein 2-like 1",
  "gene": "UniProtKB:Q5TBK1",
  "gene_symbol": "N4BP2L1",
  "term_label": "Unknown molecular function",
  "term_id": "UNKNOWN:0001"
}